{
  "term_label": "voltage-gated sodium channel complex",
  "term_id": "GO:0001518",
  "gene_name": "Sodium channel protein type 7 subunit alpha",
  "gene_symbol": "SCN7A",
  "gene": "UniProtKB:Q01118"
}